{
  "term_id": "GO:0005886",
  "gene_symbol": "BRAF",
  "term_label": "plasma membrane",
  "gene": "UniProtKB:P15056",
  "gene_name": "Serine_threonine-protein kinase B-raf"
}